regulation of interleukin-18 production [GO:0032661] (biological process) Relationships: is a type of regulation of cytokine production [GO:0001817]; regulates interleukin-18 production [GO:0032621] References: PMID:23710316 Sources: GOC:mah Also known as: regulation of IL-18 production, regulation of interleukin-18 biosynthetic process, regulation of interleukin-18 secretion Definition: Any process that modulates the frequency, rate, or extent of interleukin-18 production. Subtypes: negative regulation of interleukin-18 production [GO:0032701], positive regulation of interleukin-18 production [GO:0032741]